negative regulation of adiponectin secretion [GO:0070164] (biological process) Also known as: down regulation of adiponectin secretion, down-regulation of adiponectin secretion, downregulation of adiponectin secretion, inhibition of adiponectin secretion Sources: GOC:BHF, GOC:mah Relationships: is a type of negative regulation of hormone secretion [GO:0046888]; is a type of negative regulation of protein secretion [GO:0050709]; is a type of negative regulation of multicellular organismal process [GO:0051241]; is a type of regulation of adiponectin secretion [GO:0070163]; negatively regulates adiponectin secretion [GO:0070162] Definition: Any process that stops, prevents, or reduces the frequency, rate or extent of the regulated release of adiponectin from a cell.